{
  "gene_symbol": "DLD",
  "gene_name": "Dihydrolipoyl dehydrogenase, mitochondrial",
  "term_id": "GO:0005739",
  "gene": "UniProtKB:P09622",
  "term_label": "mitochondrion"
}